thiocyanate methyltransferase activity [GO:0102215] (molecular function) Definition: Catalysis of the reaction: thiocyanate + S-adenosyl-L-methionine = methyl thiocyanate + S-adenosyl-L-homocysteine. Sources: RHEA:28014 Relationships: is a type of methyltransferase activity [GO:0008168]